{
  "gene": "UniProtKB:Q9NRG7",
  "gene_symbol": "SDR39U1",
  "term_label": "Unknown molecular function",
  "term_id": "UNKNOWN:0001",
  "gene_name": "Epimerase family protein SDR39U1"
}